{
  "gene_name": "IQCJ-SCHIP1 readthrough transcript protein",
  "gene_symbol": "IQCJ-SCHIP1",
  "term_id": "UNKNOWN:0001",
  "gene": "UniProtKB:B3KU38",
  "term_label": "Unknown molecular function"
}